{
  "gene": "UniProtKB:Q8N5C6",
  "gene_symbol": "SRBD1",
  "term_id": "GO:0006412",
  "term_label": "translation",
  "gene_name": "S1 RNA-binding domain-containing protein 1"
}